{
  "gene_name": "Probable ATP-dependent RNA helicase DDX6",
  "gene_symbol": "DDX6",
  "term_label": "P-body assembly",
  "term_id": "GO:0033962",
  "gene": "UniProtKB:P26196"
}